{
  "term_label": "Unknown cellular component",
  "gene_name": "Fumarylacetoacetase",
  "gene_symbol": "FAH",
  "term_id": "UNKNOWN:0003",
  "gene": "UniProtKB:P16930"
}